{
  "gene_name": "Multiple epidermal growth factor-like domains protein 10",
  "term_label": "scavenger receptor activity",
  "gene": "UniProtKB:Q96KG7",
  "term_id": "GO:0005044",
  "gene_symbol": "MEGF10"
}